{
  "term_label": "sphingolipid biosynthetic process",
  "gene": "UniProtKB:Q9P035",
  "gene_symbol": "HACD3",
  "term_id": "GO:0030148",
  "gene_name": "Very-long-chain (3R)-3-hydroxyacyl-CoA dehydratase 3"
}